N-acetylglucosamine transmembrane transporter activity [GO:0015572] (MF) Also known as: D-GlcNAc transmembrane transporter activity, N-acetyl-D-glucosamine transmembrane transporter activity, N-acetylchitosamine transmembrane transporter activity, N-Acetyl-D-glucosamine permease, N-acetylglucosamine permease activity Definition: Enables the transfer of N-acetylglucosamine from one side of a membrane to the other. The D isomer of N-acetylglucosamine is a common structural unit of glycoproteins in plants, bacteria and animals; it is often the terminal sugar of an oligosaccharide group of a glycoprotein. Relationships: is a type of carbohydrate derivative transmembrane transporter activity [GO:1901505] Sources: GOC:ai, GOC:mtg_transport, ISBN:0815340729 Subtypes: GO:0022880